{
  "term_label": "Unknown biological process",
  "term_id": "UNKNOWN:0002",
  "gene_name": "Keratin-associated protein 5-1",
  "gene_symbol": "KRTAP5-1",
  "gene": "UniProtKB:Q6L8H4"
}